{
  "gene": "UniProtKB:P49184",
  "gene_name": "Deoxyribonuclease-1-like 1",
  "term_label": "deoxyribonuclease I activity",
  "gene_symbol": "DNASE1L1",
  "term_id": "GO:0004530"
}